{
  "term_label": "transcription coactivator activity",
  "gene_symbol": "MYSM1",
  "gene": "UniProtKB:Q5VVJ2",
  "term_id": "GO:0003713",
  "gene_name": "Deubiquitinase MYSM1"
}